{
  "gene_symbol": "GNG5B",
  "term_label": "G-protein beta-subunit binding",
  "gene": "UniProtKB:A0A804HLA8",
  "term_id": "GO:0031681",
  "gene_name": "Guanine nucleotide-binding protein G(I)_G(S)_G(O) subunit gamma-5B"
}